cellular response to brassinosteroid stimulus [GO:0071367] (biological process) Definition: Any process that results in a change in state or activity of a cell (in terms of movement, secretion, enzyme production, gene expression, etc.) as a result of a brassinosteroid stimulus. Relationships: is a type of response to brassinosteroid [GO:0009741]; is a type of cellular response to hormone stimulus [GO:0032870]; is_a GO:0071396; is a type of cellular response to oxygen-containing compound [GO:1901701] Sources: GOC:mah